{
  "term_id": "GO:0006099",
  "term_label": "tricarboxylic acid cycle",
  "gene_symbol": "SUCLG2",
  "gene_name": "Succinate--CoA ligase [GDP-forming] subunit beta, mitochondrial",
  "gene": "UniProtKB:Q96I99"
}